{
  "term_label": "nucleosome",
  "gene_symbol": "H2BC15",
  "term_id": "GO:0000786",
  "gene": "UniProtKB:Q99877",
  "gene_name": "Histone H2B type 1-N"
}